{
  "gene_symbol": "MPV17",
  "term_label": "Unknown biological process",
  "term_id": "UNKNOWN:0002",
  "gene": "UniProtKB:P39210",
  "gene_name": "Protein Mpv17"
}